{
  "gene_symbol": "SMIM15",
  "gene_name": "Small integral membrane protein 15",
  "term_label": "Unknown cellular component",
  "term_id": "UNKNOWN:0003",
  "gene": "UniProtKB:Q7Z3B0"
}